{
  "gene": "UniProtKB:Q86W54",
  "gene_symbol": "SPATA24",
  "term_id": "UNKNOWN:0002",
  "term_label": "Unknown biological process",
  "gene_name": "Spermatogenesis-associated protein 24"
}